{
  "term_id": "GO:0016581",
  "term_label": "NuRD complex",
  "gene": "UniProtKB:Q9BTC8",
  "gene_symbol": "MTA3",
  "gene_name": "Metastasis-associated protein MTA3"
}